{
  "gene": "UniProtKB:Q8IZU1",
  "term_id": "GO:0007286",
  "term_label": "spermatid development",
  "gene_name": "Protein FAM9A",
  "gene_symbol": "FAM9A"
}